{
  "term_id": "GO:0005765",
  "term_label": "lysosomal membrane",
  "gene_name": "HLA class II histocompatibility antigen, DO alpha chain",
  "gene_symbol": "HLA-DOA",
  "gene": "UniProtKB:P06340"
}